{
  "gene": "UniProtKB:Q99683",
  "gene_name": "Mitogen-activated protein kinase kinase kinase 5",
  "term_id": "GO:0008631",
  "gene_symbol": "MAP3K5",
  "term_label": "intrinsic apoptotic signaling pathway in response to oxidative stress"
}